1,3-dichloropropene metabolic process [GO:0018903] (BP) Sources: UM-BBD_pathwayID:cpr Definition: The chemical reactions and pathways involving members of the 1,3-dichloropropene family, which includes cis- and trans-1,3-dichloropropene. The 1,3-dichloropropenes are chlorinated hydrocarbons and the major active ingredients of commercial products for control of plant-parasitic nematodes. Also known as: 1,3-dichloropropene metabolism, 1,3-dichloropropylene metabolic process, 1,3-dichloropropylene metabolism, gamma-chloroallylchloride metabolic process, gamma-chloroallylchloride metabolism Relationships: is a type of GO:0042197